{
  "gene_name": "E3 ubiquitin-protein ligase TRIM35",
  "gene": "UniProtKB:Q9UPQ4",
  "gene_symbol": "TRIM35",
  "term_label": "cytoplasm",
  "term_id": "GO:0005737"
}